{
  "term_id": "UNKNOWN:0003",
  "gene": "UniProtKB:Q96JS3",
  "gene_symbol": "PGBD1",
  "term_label": "Unknown cellular component",
  "gene_name": "PiggyBac transposable element-derived protein 1"
}